{
  "gene": "UniProtKB:P05388",
  "gene_name": "Large ribosomal subunit protein uL10",
  "term_id": "GO:0022625",
  "gene_symbol": "RPLP0",
  "term_label": "cytosolic large ribosomal subunit"
}